negative regulation of iron export across plasma membrane [GO:1904039] (biological process) References: PMID:15514116 Sources: GOC:BHF, GOC:TermGenie, GOC:kom, GO_REF:0000058 Relationships: is a type of GO:0034760; is a type of regulation of iron export across plasma membrane [GO:1904038]; negatively regulates iron ion export across plasma membrane [GO:1903988] Also known as: down regulation of ferrous iron export, down regulation of iron(2+) export, down-regulation of ferrous iron export, down-regulation of iron(2+) export, downregulation of ferrous iron export, downregulation of iron(2+) export, inhibition of ferrous iron export, inhibition of iron(2+) export, negative regulation of ferrous iron export, negative regulation of iron(2+) export Definition: Any process that stops, prevents or reduces the frequency, rate or extent of export of iron ions from inside of a cell, across the plasma membrane and into the extracellular region.